antigen processing and presentation of peptide antigen via MHC class Ib [GO:0002428] (biological process) Also known as: peptide antigen processing and presentation via MHC class Ib Relationships: is a type of GO:0002475; is a type of antigen processing and presentation of peptide antigen [GO:0048002] Definition: The process in which an antigen-presenting cell expresses peptide antigen in association with an MHC class Ib protein complex on its cell surface. The peptide antigen may originate from an endogenous or exogenous protein. Class Ib here refers to non-classical class I molecules, such as those of the HLA-E family. Subtypes: GO:0002476, antigen processing and presentation of exogenous peptide antigen via MHC class Ib [GO:0002477] Regulation: regulated by GO:0002595; RO_0002212 by GO:0002596; positively regulated by positive regulation of antigen processing and presentation of peptide antigen via MHC class Ib [GO:0002597] References: PMID:15928678 Sources: GOC:add